{
  "term_id": "UNKNOWN:0002",
  "gene_name": "RNA-binding protein with multiple splicing",
  "gene_symbol": "RBPMS",
  "term_label": "Unknown biological process",
  "gene": "UniProtKB:Q93062"
}